{
  "term_label": "nucleus",
  "gene": "UniProtKB:Q9Y5R6",
  "gene_symbol": "DMRT1",
  "gene_name": "Doublesex- and mab-3-related transcription factor 1",
  "term_id": "GO:0005634"
}